{
  "term_label": "signal transduction",
  "gene_symbol": "GRAP",
  "gene_name": "GRB2-related adapter protein",
  "gene": "UniProtKB:Q13588",
  "term_id": "GO:0007165"
}